{
  "term_label": "Unknown molecular function",
  "gene_name": "Putative uncharacterized protein FLJ92257",
  "gene": "UniProtKB:Q75L30",
  "term_id": "UNKNOWN:0001",
  "gene_symbol": "Q75L30"
}